Renilla-luciferin sulfotransferase activity [GO:0050249] (MF) Relationships: is a type of GO:0008146 Also known as: luciferin sulfotransferase activity, Renilla-luciferin sulphotransferase activity, 3'-phosphoadenylyl-sulfate:Renilla luciferin sulfotransferase activity, luciferin sulfokinase (3'-phosphoadenylyl sulfate:luciferin sulfotransferase), luciferin sulfokinase activity Definition: Catalysis of the reaction: 3'-phospho-5'-adenylyl sulfate + Renilla luciferin = adenosine 3',5'-diphosphate + H+ + luciferyl sulfate. Sources: EC:2.8.2.10, RHEA:20481